nuclear estrogen receptor activity [GO:0030284] (molecular function) Definition: A nuclear receptor activity regulated by estrogen binding and modulating the transcription of specific gene sets transcribed by RNA polymerase II. Also known as: estrogen receptor activity References: PMID:17615392 Sources: GOC:signaling Relationships: is a type of GO:0003707